{
  "gene_symbol": "RBMS2",
  "gene": "UniProtKB:Q15434",
  "gene_name": "RNA-binding motif, single-stranded-interacting protein 2",
  "term_label": "mRNA 3'-UTR binding",
  "term_id": "GO:0003730"
}